tricellular tight junction disassembly [GO:1904275] (biological process) Relationships: is a type of GO:1905071 Definition: The disaggregation of a tricellular tight junction into its constituent components. References: PMID:22640933, PMID:25097825, PMID:4203962 Sources: GOC:TermGenie, GOC:mr, GO_REF:0000079